forebrain radial glial cell differentiation [GO:0021861] (biological process) Also known as: radial glial cell differentiation in forebrain Relationships: is a type of radial glial cell differentiation [GO:0060019]; is part of forebrain generation of neurons [GO:0021872] Definition: The process in which neuroepithelial cells of the neural tube give rise to radial glial cells, specialized bipotential progenitors cells of the forebrain. Differentiation includes the processes involved in commitment of a cell to a specific fate. References: PMID:16226447 Sources: GOC:cls, GOC:dgh, GOC:dph, GOC:jid, GO_REF:0000021